rRNA (guanine-N7)-methylation [GO:0070476] (biological process) Sources: GOC:mah Definition: The addition of a methyl group to the N7 atom in the base portion of a guanine nucleotide residue in an rRNA molecule. Relationships: is a type of GO:0036265; is a type of rRNA base methylation [GO:0070475]